{
  "term_id": "UNKNOWN:0001",
  "gene_symbol": "SLITRK2",
  "gene_name": "SLIT and NTRK-like protein 2",
  "gene": "UniProtKB:Q9H156",
  "term_label": "Unknown molecular function"
}